{
  "term_label": "Unknown biological process",
  "term_id": "UNKNOWN:0002",
  "gene": "UniProtKB:Q96I45",
  "gene_symbol": "TMEM141",
  "gene_name": "Transmembrane protein 141"
}